histone decrotonylase activity [GO:0160009] (molecular function) Subtypes: GO:0160012 References: PMID:28497810 Relationships: is a type of histone modifying activity [GO:0140993]; is a type of protein decrotonylase activity [GO:0160008] Definition: Catalysis of the reaction: H2O + N6-(2E)-butenoyl-L-lysyl-[histone] = (2E)-2-butenoate + L-lysyl-[histone].